{
  "gene_symbol": "NT5C1B",
  "gene_name": "Cytosolic 5'-nucleotidase 1B",
  "term_label": "5'-nucleotidase activity",
  "term_id": "GO:0008253",
  "gene": "UniProtKB:Q96P26"
}